{
  "gene": "UniProtKB:P60852",
  "gene_symbol": "ZP1",
  "term_id": "GO:0035805",
  "term_label": "egg coat",
  "gene_name": "Zona pellucida sperm-binding protein 1"
}